{
  "gene_name": "Sodium-dependent proline transporter",
  "gene": "UniProtKB:Q99884",
  "term_label": "plasma membrane",
  "term_id": "GO:0005886",
  "gene_symbol": "SLC6A7"
}